{
  "gene_name": "Glutathione peroxidase 7",
  "term_label": "Unknown cellular component",
  "term_id": "UNKNOWN:0003",
  "gene": "UniProtKB:Q96SL4",
  "gene_symbol": "GPX7"
}